{
  "term_id": "GO:0045338",
  "term_label": "farnesyl diphosphate metabolic process",
  "gene": "UniProtKB:P37268",
  "gene_name": "Squalene synthase",
  "gene_symbol": "FDFT1"
}